{
  "gene_symbol": "SSU72L3",
  "gene": "UniProtKB:A0A1W2PQJ5",
  "term_label": "termination of RNA polymerase II transcription",
  "term_id": "GO:0006369",
  "gene_name": "RNA polymerase II subunit A C-terminal domain phosphatase SSU72 like protein 3"
}